cytokinin metabolic process [GO:0009690] (BP) Definition: The chemical reactions and pathways involving cytokinins, a class of adenine-derived compounds that can function in plants as growth regulators. Sources: ISBN:0387969845 Also known as: cytokinin metabolism Subtypes: cytokinin biosynthetic process [GO:0009691], cytokinin catabolic process [GO:0009823] Relationships: is a type of GO:0009308; is a type of hormone metabolic process [GO:0042445]